{
  "gene_name": "Killer cell immunoglobulin-like receptor, three Ig domains pseudogene 1",
  "term_id": "GO:0004888",
  "gene": "UniProtKB:A0A0G2JN01",
  "gene_symbol": "KIR3DP1",
  "term_label": "transmembrane signaling receptor activity"
}